negative regulation of isopentenyl diphosphate biosynthetic process, mevalonate pathway [GO:2001211] (biological process) Also known as: negative regulation of Ac-MVA pathway, negative regulation of acetate-mevalonate pathway, negative regulation of isopentenyl diphosphate anabolism, mevalonate pathway, negative regulation of isopentenyl diphosphate formation, mevalonate pathway, negative regulation of isopentenyl diphosphate synthesis, mevalonate pathway Definition: Any process that stops, prevents or reduces the frequency, rate or extent of isopentenyl diphosphate biosynthetic process, mevalonate pathway. Sources: GOC:al Relationships: is a type of negative regulation of amide metabolic process [GO:0034249]; is_a negative regulation of isoprenoid metabolic process [GO:0045827]; is a type of negative regulation of nucleobase-containing compound metabolic process [GO:0045934]; is a type of negative regulation of small molecule metabolic process [GO:0062014]; is a type of negative regulation of phospholipid biosynthetic process [GO:0071072]; is a type of regulation of isopentenyl diphosphate biosynthetic process, mevalonate pathway [GO:2001210]; negatively regulates GO:0019287